{
  "gene_name": "Whirlin",
  "term_label": "auditory receptor cell stereocilium organization",
  "gene_symbol": "WHRN",
  "term_id": "GO:0060088",
  "gene": "UniProtKB:Q9P202"
}